{
  "gene_symbol": "MANF",
  "term_label": "Unknown molecular function",
  "gene": "UniProtKB:P55145",
  "term_id": "UNKNOWN:0001",
  "gene_name": "Mesencephalic astrocyte-derived neurotrophic factor"
}